{
  "gene": "UniProtKB:Q9H7L9",
  "gene_symbol": "SUDS3",
  "term_label": "Sin3-type complex",
  "gene_name": "Sin3 histone deacetylase corepressor complex component SDS3",
  "term_id": "GO:0070822"
}